{
  "gene": "UniProtKB:A0A8I5QJS6",
  "term_id": "UNKNOWN:0001",
  "term_label": "Unknown molecular function",
  "gene_symbol": "A0A8I5QJS6",
  "gene_name": "Uncharacterized protein"
}